{
  "gene_name": "Receptor expression-enhancing protein 2",
  "gene_symbol": "REEP2",
  "term_label": "cytoplasmic microtubule",
  "gene": "UniProtKB:Q9BRK0",
  "term_id": "GO:0005881"
}